{
  "term_label": "ubiquitin-dependent protein catabolic process via the N-end rule pathway",
  "term_id": "GO:0071596",
  "gene": "UniProtKB:Q8IWV7",
  "gene_symbol": "UBR1",
  "gene_name": "E3 ubiquitin-protein ligase UBR1"
}